{
  "term_label": "Unknown molecular function",
  "gene": "UniProtKB:P20618",
  "gene_symbol": "PSMB1",
  "gene_name": "Proteasome subunit beta type-1",
  "term_id": "UNKNOWN:0001"
}